{
  "gene_name": "Rho GTPase-activating protein 28",
  "term_id": "GO:0005096",
  "gene": "UniProtKB:Q9P2N2",
  "term_label": "GTPase activator activity",
  "gene_symbol": "ARHGAP28"
}